{
  "gene_symbol": "ZNF891",
  "gene_name": "Zinc finger protein 891",
  "gene": "UniProtKB:A8MT65",
  "term_label": "DNA-binding transcription factor activity, RNA polymerase II-specific",
  "term_id": "GO:0000981"
}